{
  "term_id": "GO:0031519",
  "term_label": "PcG protein complex",
  "gene": "UniProtKB:Q06587",
  "gene_symbol": "RING1",
  "gene_name": "E3 ubiquitin-protein ligase RING1"
}